{
  "gene": "UniProtKB:A6NGU5",
  "gene_name": "Putative glutathione hydrolase 3 proenzyme",
  "term_label": "regulation of immune system process",
  "term_id": "GO:0002682",
  "gene_symbol": "GGT3P"
}